{
  "gene_symbol": "OR52E4",
  "gene": "UniProtKB:Q8NGH9",
  "term_label": "Unknown biological process",
  "gene_name": "Olfactory receptor 52E4",
  "term_id": "UNKNOWN:0002"
}